{
  "term_label": "microtubule binding",
  "gene_symbol": "SPIRE1",
  "gene": "UniProtKB:Q08AE8",
  "term_id": "GO:0008017",
  "gene_name": "Protein spire homolog 1"
}